{
  "gene_symbol": "CEMIP2",
  "gene_name": "Cell surface hyaluronidase",
  "gene": "UniProtKB:Q9UHN6",
  "term_id": "UNKNOWN:0001",
  "term_label": "Unknown molecular function"
}